{
  "gene_name": "Chemokine-like protein TAFA-1",
  "term_label": "neuroblast differentiation",
  "gene_symbol": "TAFA1",
  "gene": "UniProtKB:Q7Z5A9",
  "term_id": "GO:0014016"
}